{
  "gene_name": "Caveolin-3",
  "term_id": "GO:0044325",
  "gene_symbol": "CAV3",
  "gene": "UniProtKB:P56539",
  "term_label": "transmembrane transporter binding"
}